regulation of defense response to fungus [GO:1900150] (biological process) References: PMID:22242006 Sources: GOC:TermGenie, GOC:dhl Definition: Any process that modulates the frequency, rate or extent of defense response to fungus. Relationships: is a type of regulation of response to biotic stimulus [GO:0002831]; is a type of regulation of defense response [GO:0031347]; is a type of regulation of response to external stimulus [GO:0032101]; regulates defense response to fungus [GO:0050832] Also known as: regulation of defence response to fungi, regulation of defence response to fungus, regulation of defense response to fungi, regulation of defense response to fungi, incompatible interaction, regulation of defense response to fungus, incompatible interaction, regulation of resistance response to pathogenic fungi, regulation of resistance response to pathogenic fungus, regulation of response to pathogenic fungus (incompatible interaction) Subtypes: regulation of antifungal peptide production [GO:0002788], regulation of neutrophil mediated killing of fungus [GO:0070953], GO:1905034